regulation of retinal cone cell fate specification [GO:0042673] (biological process) Definition: Any process that mediates the specification of a cell into a retinal cone cell. Subtypes: negative regulation of retinal cone cell fate specification [GO:0009998] Relationships: is a type of regulation of cell fate specification [GO:0042659]; is a type of regulation of retinal cone cell fate commitment [GO:0060222]; regulates retinal cone cell fate specification [GO:0042672] Sources: GOC:go_curators